{
  "term_label": "plasma membrane",
  "gene": "UniProtKB:A1L1A6",
  "gene_symbol": "IGSF23",
  "term_id": "GO:0005886",
  "gene_name": "Immunoglobulin superfamily member 23"
}